{
  "gene_symbol": "SLC35E2A",
  "gene_name": "Solute carrier family 35 member E2A",
  "term_label": "transmembrane transport",
  "term_id": "GO:0055085",
  "gene": "UniProtKB:P0CK97"
}